{
  "gene": "UniProtKB:Q9BQG1",
  "gene_name": "Synaptotagmin-3",
  "term_id": "GO:0005544",
  "term_label": "calcium-dependent phospholipid binding",
  "gene_symbol": "SYT3"
}